nephrogenic mesenchyme morphogenesis [GO:0072134] (biological process) Sources: GOC:mtg_kidney_jan10 Relationships: is a type of kidney mesenchyme morphogenesis [GO:0072131]; is part of GO:0072076 Definition: The process in which the anatomical structures of a nephrogenic mesenchymal tissue are generated and organized. Nephrogenic mesenchyme is the tissue made up of loosely connected mesenchymal cells in the nephron.